{
  "gene_name": "Transmembrane and coiled-coil domain-containing protein 3",
  "gene_symbol": "TMCO3",
  "gene": "UniProtKB:Q6UWJ1",
  "term_id": "UNKNOWN:0003",
  "term_label": "Unknown cellular component"
}